{
  "term_id": "GO:0008143",
  "gene_name": "Polyadenylate-binding protein 4-like",
  "gene": "UniProtKB:P0CB38",
  "term_label": "poly(A) binding",
  "gene_symbol": "PABPC4L"
}